{
  "term_label": "U4 snRNP",
  "gene_name": "Small nuclear ribonucleoprotein E",
  "gene": "UniProtKB:P62304",
  "term_id": "GO:0005687",
  "gene_symbol": "SNRPE"
}